L-cysteine catabolic process to taurine [GO:0019452] (biological process) Definition: The chemical reactions and pathways resulting in the breakdown of L-cysteine into other compounds, including taurine. Also known as: L-cysteine breakdown to taurine, L-cysteine degradation to taurine Relationships: is a type of L-cysteine catabolic process [GO:0019448]; is a type of taurine metabolic process [GO:0019530] Sources: GOC:go_curators